{
  "term_label": "Unknown biological process",
  "term_id": "UNKNOWN:0002",
  "gene": "UniProtKB:P62841",
  "gene_name": "Small ribosomal subunit protein uS19",
  "gene_symbol": "RPS15"
}